{
  "gene_symbol": "RIPK2",
  "term_id": "GO:0004706",
  "gene": "UniProtKB:O43353",
  "term_label": "JUN kinase kinase kinase activity",
  "gene_name": "Receptor-interacting serine_threonine-protein kinase 2"
}